{
  "term_label": "HCN channel complex",
  "gene": "UniProtKB:Q9Y3Q4",
  "gene_symbol": "HCN4",
  "term_id": "GO:0098855",
  "gene_name": "Potassium_sodium hyperpolarization-activated cyclic nucleotide-gated channel 4"
}